{
  "term_id": "GO:0000122",
  "term_label": "negative regulation of transcription by RNA polymerase II",
  "gene": "UniProtKB:P12755",
  "gene_name": "Ski oncogene",
  "gene_symbol": "SKI"
}